{
  "gene_name": "Retinal rod rhodopsin-sensitive cGMP 3',5'-cyclic phosphodiesterase subunit gamma",
  "gene": "UniProtKB:P18545",
  "term_label": "positive regulation of G protein-coupled receptor signaling pathway",
  "gene_symbol": "PDE6G",
  "term_id": "GO:0045745"
}